regulation of long-day photoperiodism, flowering [GO:0048586] (BP) Sources: GOC:jid, GOC:pj, ISBN:0582015952, ISBN:0697037754, ISBN:0709408862 Relationships: is a type of regulation of photoperiodism, flowering [GO:2000028]; regulates GO:0048574 Subtypes: positive regulation of long-day photoperiodism, flowering [GO:0048578], negative regulation of long-day photoperiodism, flowering [GO:0048579] Definition: Any process that modulates the frequency, rate or extent of long-day photoperiodism, where the response associated with the photoperiodism is flowering. Flowering is defined by the switch from the vegetative to the reproductive phase.